{
  "term_label": "Unknown cellular component",
  "term_id": "UNKNOWN:0003",
  "gene": "UniProtKB:Q75N03",
  "gene_symbol": "CBLL1",
  "gene_name": "E3 ubiquitin-protein ligase Hakai"
}